negative regulation of epithelial to mesenchymal transition involved in endocardial cushion formation [GO:1905006] (biological process) Also known as: down regulation of epithelial to mesenchymal transition involved in endocardial cushion formation, down-regulation of epithelial to mesenchymal transition involved in endocardial cushion formation, downregulation of epithelial to mesenchymal transition involved in endocardial cushion formation, inhibition of epithelial to mesenchymal transition involved in endocardial cushion formation Relationships: is a type of negative regulation of cardiac epithelial to mesenchymal transition [GO:0062044]; is a type of regulation of epithelial to mesenchymal transition involved in endocardial cushion formation [GO:1905005]; negatively regulates GO:0003198 Definition: Any process that stops, prevents or reduces the frequency, rate or extent of epithelial to mesenchymal transition involved in endocardial cushion formation. References: PMID:18718461 Sources: GOC:BHF, GOC:TermGenie, GOC:rl, GO_REF:0000058